nucleoplasmic periphery of the nuclear pore complex [GO:1990826] (cellular component) Also known as: associated with the nuclear pore Definition: Nucleoplasm situated in close proximity and peripheral to a nuclear pore complex. Relationships: is a type of GO:0110165; is part of nucleoplasm [GO:0005654] References: PMID:10633080